negative regulation of natural killer cell apoptotic process [GO:0070248] (biological process) Also known as: down regulation of natural killer cell apoptosis, down-regulation of natural killer cell apoptosis, downregulation of natural killer cell apoptosis, negative regulation of NK cell apoptosis, inhibition of natural killer cell apoptosis, negative regulation of natural killer cell apoptosis Definition: Any process that stops, prevents, or reduces the frequency, rate or extent of natural killer cell death by apoptotic process. Sources: GOC:add, GOC:mtg_apoptosis, ISBN:0781765196 Relationships: is a type of negative regulation of lymphocyte apoptotic process [GO:0070229]; is a type of regulation of natural killer cell apoptotic process [GO:0070247]; negatively regulates natural killer cell apoptotic process [GO:0070246]